{
  "gene_symbol": "TIMP1",
  "term_label": "response to cytokine",
  "gene": "UniProtKB:P01033",
  "term_id": "GO:0034097",
  "gene_name": "Metalloproteinase inhibitor 1"
}